{
  "gene_name": "Transcriptional enhancer factor TEF-5",
  "gene": "UniProtKB:Q99594",
  "term_label": "DNA-binding transcription factor activity, RNA polymerase II-specific",
  "term_id": "GO:0000981",
  "gene_symbol": "TEAD3"
}